{
  "term_label": "Unknown molecular function",
  "gene": "UniProtKB:Q8N961",
  "gene_name": "Ankyrin repeat and BTB_POZ domain-containing protein 2",
  "gene_symbol": "ABTB2",
  "term_id": "UNKNOWN:0001"
}